{
  "gene": "UniProtKB:Q8IUN9",
  "term_label": "external side of plasma membrane",
  "gene_symbol": "CLEC10A",
  "gene_name": "C-type lectin domain family 10 member A",
  "term_id": "GO:0009897"
}